stamen structural organization [GO:0048456] (biological process) Definition: The process that contributes to the act of creating the structural organization of the stamen. This process pertains to the physical shaping of a rudimentary structure. Sources: GOC:jid Relationships: is_a GO:0048450; is part of stamen morphogenesis [GO:0048448] Also known as: stamen structural organisation